{
  "term_id": "UNKNOWN:0002",
  "gene": "UniProtKB:Q96DR5",
  "term_label": "Unknown biological process",
  "gene_symbol": "BPIFA2",
  "gene_name": "BPI fold-containing family A member 2"
}